negative regulation of toll-like receptor 11 signaling pathway [GO:0034172] (biological process) Definition: Any process that stops, prevents, or reduces the frequency, rate, or extent of toll-like receptor 11 signaling pathway. References: PMID:16551253, PMID:17328678 Sources: GOC:add Relationships: is a type of regulation of toll-like receptor 11 signaling pathway [GO:0034171]; is a type of GO:0039532; negatively regulates toll-like receptor 11 signaling pathway [GO:0034170] Also known as: negative regulation of TLR11 signaling pathway, negative regulation of toll-like receptor 11 signalling pathway